regulation of formation of translation initiation ternary complex [GO:1901190] (biological process) Relationships: is a type of GO:0043254; regulates GO:0001677 Definition: Any process that modulates the frequency, rate or extent of formation of translation initiation ternary complex. Sources: GOC:TermGenie Also known as: regulation of translation initiation ternary complex assembly Subtypes: GO:1901191, positive regulation of formation of translation initiation ternary complex [GO:1901192]